{
  "term_id": "GO:0019899",
  "gene_name": "UDP-glucuronosyltransferase 1A8",
  "gene_symbol": "UGT1A8",
  "term_label": "enzyme binding",
  "gene": "UniProtKB:Q9HAW9"
}